{
  "gene_name": "Potassium channel subfamily K member 5",
  "term_label": "potassium ion transmembrane transport",
  "gene_symbol": "KCNK5",
  "term_id": "GO:0071805",
  "gene": "UniProtKB:O95279"
}